{
  "term_id": "GO:0005886",
  "gene_symbol": "TSHR",
  "gene_name": "Thyrotropin receptor",
  "term_label": "plasma membrane",
  "gene": "UniProtKB:P16473"
}